{
  "term_id": "GO:0030968",
  "gene": "UniProtKB:O76024",
  "gene_name": "Wolframin",
  "gene_symbol": "WFS1",
  "term_label": "endoplasmic reticulum unfolded protein response"
}